dense body [GO:0097433] (cellular component) Definition: An electron dense body which may contain granules. Relationships: is a type of GO:0110165; is part of cytoplasm [GO:0005737] Sources: ISBN:0195065719, NIF_Subcellular:sao730872736